lipid A metabolic process [GO:0046493] (biological process) Also known as: lipid A metabolism References: PMID:20974832, PMID:22216004 Sources: ISBN:0198506732 Subtypes: lipid A biosynthetic process [GO:0009245] Relationships: is a type of GO:0006644; is a type of glycolipid metabolic process [GO:0006664]; is a type of lipooligosaccharide metabolic process [GO:1901269] Definition: The chemical reactions and pathways involving lipid A, the glycolipid group of bacterial lipopolysaccharides, consisting of four to six fatty acyl chains linked to two glucosamine residues. Further modifications of the backbone are common.